{
  "term_label": "IgG binding",
  "term_id": "GO:0019864",
  "gene": "UniProtKB:P31994",
  "gene_name": "Low affinity immunoglobulin gamma Fc region receptor II-b",
  "gene_symbol": "FCGR2B"
}